{
  "gene": "UniProtKB:Q8WUB8",
  "gene_symbol": "PHF10",
  "gene_name": "PHD finger protein 10",
  "term_label": "chromatin binding",
  "term_id": "GO:0003682"
}